regulation of store-operated calcium channel activity [GO:1901339] (biological process) Subtypes: negative regulation of store-operated calcium channel activity [GO:1901340], positive regulation of store-operated calcium channel activity [GO:1901341] Sources: GOC:TermGenie Definition: Any process that modulates the frequency, rate or extent of store-operated calcium channel activity. Relationships: is a type of GO:0022898; regulates store-operated calcium channel activity [GO:0015279]